{
  "gene": "UniProtKB:Q8MH63",
  "term_label": "Unknown molecular function",
  "gene_symbol": "SLC7A5P1",
  "gene_name": "Putative L-type amino acid transporter 1-like protein MLAS",
  "term_id": "UNKNOWN:0001"
}